{
  "gene_symbol": "CTNNB1",
  "gene_name": "Catenin beta-1",
  "gene": "UniProtKB:P35222",
  "term_id": "GO:0019903",
  "term_label": "protein phosphatase binding"
}